entry into host cell by a symbiont-containing vacuole [GO:0085017] (biological process) Definition: The invasion by a symbiont of a cell of a host organism, forming a vacuole in which the symbiont resides. The vacuole membrane is formed from lipids and proteins derived from both host and symbiont. Begins when the symbiont attaches on to the host cell membrane which invaginates and deepens as the symbiont enters, and ends when the host cell membrane closes behind the newly-formed vacuole. References: PMID:18665841, PMID:8690024, PMID:9580555 Sources: GOC:jl Also known as: symbiont entry into host cell forming a parasitophorous vacuole, symbiont entry into host cell forming a pathogen-containing vacuole, symbiont entry into host cell forming a symbiont-containing vacuole Relationships: is_a symbiont entry into host cell [GO:0046718]